regulation of viral transcription [GO:0046782] (biological process) Sources: GOC:ai Relationships: is a type of regulation of viral process [GO:0050792]; RO_0002211 GO:0019083 Definition: Any process that modulates the frequency, rate or extent of the transcription of the viral genome. Subtypes: negative regulation of viral transcription [GO:0032897], positive regulation of viral transcription [GO:0050434]